{
  "gene": "UniProtKB:Q6ZTQ4",
  "gene_symbol": "CDHR3",
  "term_label": "catenin complex",
  "term_id": "GO:0016342",
  "gene_name": "Cadherin-related family member 3"
}